histone-dependent DNA binding [GO:0099077] (molecular function) Relationships: is_a GO:0003677 References: PMID:11691835 Definition: DNA-binding activity that is dependent on binding to a histone.